{
  "gene_symbol": "ZNF43",
  "gene": "UniProtKB:P17038",
  "term_label": "nucleus",
  "term_id": "GO:0005634",
  "gene_name": "Zinc finger protein 43"
}